{
  "gene_symbol": "CLCN2",
  "gene": "UniProtKB:P51788",
  "term_id": "GO:0006821",
  "term_label": "chloride transport",
  "gene_name": "Chloride channel protein 2"
}